{
  "gene_symbol": "TMEM223",
  "term_id": "UNKNOWN:0001",
  "gene_name": "Transmembrane protein 223",
  "gene": "UniProtKB:A0PJW6",
  "term_label": "Unknown molecular function"
}